nitrile catabolic process [GO:0050899] (biological process) Definition: The chemical reactions and pathways resulting in the breakdown of a nitrile, an organic compound containing trivalent nitrogen attached to one carbon atom. Sources: ISBN:0721662544 Also known as: nitrile breakdown, nitrile catabolism, nitrile degradation Relationships: is a type of catabolic process [GO:0009056]; is a type of nitrile metabolic process [GO:0050898] Subtypes: GO:0019256, GO:0042342, 3-cyano-L-alanine catabolic process [GO:1903559]